{
  "term_id": "GO:0007098",
  "term_label": "centrosome cycle",
  "gene_name": "HEPACAM family member 2",
  "gene_symbol": "HEPACAM2",
  "gene": "UniProtKB:A8MVW5"
}